{
  "term_label": "nucleolus",
  "gene_symbol": "NUSAP1",
  "term_id": "GO:0005730",
  "gene_name": "Nucleolar and spindle-associated protein 1",
  "gene": "UniProtKB:Q9BXS6"
}